hyperosmotic response [GO:0006972] (biological process) Also known as: HOG response, hypertonic response, response to hypertonicity Subtypes: hyperosmotic salinity response [GO:0042538], cellular hyperosmotic response [GO:0071474] References: PMID:12142009 Sources: GOC:jl Relationships: is a type of response to osmotic stress [GO:0006970] Definition: Any process that results in a change in state or activity of a cell or an organism (in terms of movement, secretion, enzyme production, gene expression, etc.) as a result of detection of, or exposure to, a hyperosmotic environment, i.e. an environment with a higher concentration of solutes than the organism or cell.